{
  "gene_symbol": "PCNX2",
  "term_label": "Unknown biological process",
  "term_id": "UNKNOWN:0002",
  "gene": "UniProtKB:A6NKB5",
  "gene_name": "Pecanex-like protein 2"
}